{
  "gene_symbol": "IGKJ1",
  "term_label": "Unknown biological process",
  "gene": "UniProtKB:A0A0A0MT89",
  "gene_name": "Immunoglobulin kappa joining 1",
  "term_id": "UNKNOWN:0002"
}